{
  "term_id": "GO:0010669",
  "gene_symbol": "FREM1",
  "gene_name": "FRAS1-related extracellular matrix protein 1",
  "term_label": "epithelial structure maintenance",
  "gene": "UniProtKB:Q5H8C1"
}